{
  "term_id": "GO:0005635",
  "gene_symbol": "FBXW11",
  "gene": "UniProtKB:Q9UKB1",
  "term_label": "nuclear envelope",
  "gene_name": "F-box_WD repeat-containing protein 11"
}